{
  "gene_name": "Endophilin-B2",
  "gene": "UniProtKB:Q9NR46",
  "term_id": "GO:0061024",
  "gene_symbol": "SH3GLB2",
  "term_label": "membrane organization"
}